heme B biosynthetic process [GO:0006785] (BP) References: PMID:29414780 Sources: GOC:yaf Definition: The chemical reactions and pathways resulting in the formation of heme B, a Fe(II) porphyrin complex readily isolated from the hemoglobin of beef blood, but also found in other proteins including other hemoglobins, myoglobins, cytochromes P-450, catalases, peroxidases as well as b type cytochromes. Also known as: haem B biosynthesis, haem B biosynthetic process, heme B anabolism, heme B biosynthesis, heme B formation, heme B synthesis, protoheme biosynthesis, protoheme biosynthetic process Relationships: is a type of GO:0006783